methionine biosynthetic process [GO:0009086] (biological process) Relationships: is a type of GO:0000097; is a type of GO:0006555; is_a aspartate family amino acid biosynthetic process [GO:0009067] Also known as: methionine anabolism, methionine biosynthesis, methionine formation, methionine synthesis Subtypes: L-methionine biosynthetic process [GO:0071265] Definition: The chemical reactions and pathways resulting in the formation of methionine (2-amino-4-(methylthio)butanoic acid), a sulfur-containing, essential amino acid found in peptide linkage in proteins. Sources: GOC:jl, ISBN:0198506732